{
  "gene_name": "Phospholipase D2",
  "term_label": "phospholipase D activity",
  "term_id": "GO:0004630",
  "gene_symbol": "PLD2",
  "gene": "UniProtKB:O14939"
}